{
  "term_label": "nucleoplasm",
  "term_id": "GO:0005654",
  "gene_symbol": "CENPW",
  "gene_name": "Centromere protein W",
  "gene": "UniProtKB:Q5EE01"
}